circadian sleep/wake cycle process [GO:0022410] (biological process) Definition: A behavioral process involved in the cycle from wakefulness through an orderly succession of sleep states and stages that occurs on an approximately 24 hour rhythm. Relationships: is a type of circadian behavior [GO:0048512]; is part of circadian sleep/wake cycle [GO:0042745] Subtypes: circadian sleep/wake cycle, wakefulness [GO:0042746], circadian sleep/wake cycle, REM sleep [GO:0042747], GO:0042748, circadian sleep/wake cycle, sleep [GO:0050802] Sources: GOC:isa_complete